{
  "term_id": "UNKNOWN:0002",
  "gene_name": "Protein FAM47B",
  "gene_symbol": "FAM47B",
  "term_label": "Unknown biological process",
  "gene": "UniProtKB:Q8NA70"
}